{
  "gene_name": "Neuronal vesicle trafficking-associated protein 1",
  "term_label": "endosome",
  "gene": "UniProtKB:P42857",
  "term_id": "GO:0005768",
  "gene_symbol": "NSG1"
}